negative regulation of collagen catabolic process [GO:0010711] (BP) Also known as: down regulation of collagen catabolic process, down-regulation of collagen catabolic process, downregulation of collagen catabolic process, negative regulation of collagen breakdown, negative regulation of collagen catabolism, negative regulation of collagen degradation, inhibition of collagen catabolic process Definition: Any process that decreases the rate, frequency or extent of collagen catabolism. Collagen catabolism is the proteolytic chemical reactions and pathways resulting in the breakdown of collagen in the extracellular matrix. Sources: GOC:BHF, GOC:dph, GOC:tb Relationships: is a type of negative regulation of catabolic process [GO:0009895]; is a type of GO:0010710; is a type of negative regulation of collagen metabolic process [GO:0010713]; negatively regulates collagen catabolic process [GO:0030574]